{
  "gene_symbol": "ACADVL",
  "gene_name": "Very long-chain specific acyl-CoA dehydrogenase, mitochondrial",
  "term_label": "fatty-acyl-CoA binding",
  "gene": "UniProtKB:P49748",
  "term_id": "GO:0000062"
}